{
  "gene_symbol": "TIRAP",
  "term_label": "toll-like receptor 4 signaling pathway",
  "term_id": "GO:0034142",
  "gene": "UniProtKB:P58753",
  "gene_name": "Toll_interleukin-1 receptor domain-containing adapter protein"
}